{
  "gene_name": "SLAIN motif-containing protein 1",
  "term_label": "positive regulation of microtubule polymerization",
  "term_id": "GO:0031116",
  "gene": "UniProtKB:Q8ND83",
  "gene_symbol": "SLAIN1"
}